{
  "gene_symbol": "LYN",
  "term_id": "GO:0007169",
  "gene_name": "Tyrosine-protein kinase Lyn",
  "term_label": "cell surface receptor protein tyrosine kinase signaling pathway",
  "gene": "UniProtKB:P07948"
}